{
  "gene_symbol": "OLFML2B",
  "gene": "UniProtKB:Q68BL8",
  "term_id": "UNKNOWN:0001",
  "term_label": "Unknown molecular function",
  "gene_name": "Olfactomedin-like protein 2B"
}